{
  "term_label": "protein tyrosine phosphatase activity",
  "term_id": "GO:0004725",
  "gene_symbol": "PTPRO",
  "gene_name": "Receptor-type tyrosine-protein phosphatase O",
  "gene": "UniProtKB:Q16827"
}